regulation of antifungal peptide production [GO:0002788] (biological process) Subtypes: negative regulation of antifungal peptide production [GO:0002789], regulation of antifungal peptide secretion [GO:0002800], positive regulation of antifungal peptide production [GO:0002804], GO:0002810 Sources: GOC:add Relationships: is a type of regulation of antimicrobial peptide production [GO:0002784]; is a type of regulation of defense response to fungus [GO:1900150]; regulates GO:0002781 Definition: Any process that modulates the frequency, rate, or extent of antifungal peptide production.